{
  "gene_symbol": "TIMM10",
  "term_id": "GO:0042721",
  "gene": "UniProtKB:P62072",
  "term_label": "TIM22 mitochondrial import inner membrane insertion complex",
  "gene_name": "Mitochondrial import inner membrane translocase subunit Tim10"
}